{
  "gene": "UniProtKB:P53677",
  "gene_symbol": "AP3M2",
  "gene_name": "AP-3 complex subunit mu-2",
  "term_id": "GO:0006897",
  "term_label": "endocytosis"
}